{
  "gene": "UniProtKB:Q9Y6Q6",
  "gene_symbol": "TNFRSF11A",
  "term_id": "GO:0045780",
  "term_label": "positive regulation of bone resorption",
  "gene_name": "Tumor necrosis factor receptor superfamily member 11A"
}